{
  "gene_symbol": "CTXN3",
  "gene_name": "Cortexin-3",
  "term_id": "UNKNOWN:0001",
  "gene": "UniProtKB:Q4LDR2",
  "term_label": "Unknown molecular function"
}